{
  "gene_name": "Secretory carrier-associated membrane protein 3",
  "gene": "UniProtKB:O14828",
  "term_label": "Unknown molecular function",
  "term_id": "UNKNOWN:0001",
  "gene_symbol": "SCAMP3"
}